{
  "term_label": "chemokine activity",
  "gene": "UniProtKB:Q99731",
  "term_id": "GO:0008009",
  "gene_name": "C-C motif chemokine 19",
  "gene_symbol": "CCL19"
}